response to 1-aminocyclopropane-1-carboxylic acid [GO:0009961] (biological process) Definition: Any process that results in a change in state or activity of a cell or an organism (in terms of movement, secretion, enzyme production, gene expression, etc.) as a result of a 1-aminocyclopropane-1-carboxylic acid stimulus. Relationships: is a type of response to amino acid [GO:0043200]; is a type of GO:1901698; is a type of response to oxygen-containing compound [GO:1901700] Sources: GOC:jl Subtypes: cellular response to 1-aminocyclopropane-1-carboxylic acid [GO:0071213]